{
  "gene": "UniProtKB:Q7L266",
  "gene_symbol": "ASRGL1",
  "term_label": "L-asparagine catabolic process via L-aspartate",
  "term_id": "GO:0033345",
  "gene_name": "Isoaspartyl peptidase_L-asparaginase"
}